transforming growth factor beta receptor complex assembly [GO:0007181] (biological process) Also known as: TGF-beta receptor complex assembly, TGF-beta:type II receptor:type I receptor complex assembly, TGFbeta receptor complex assembly Definition: The aggregation, arrangement and bonding together of a ligand-bound type II transforming growth factor beta (TGF-beta) receptor dimer with a type I TGF-beta receptor dimer, following ligand binding, to form a heterotetrameric TGF-beta receptor complex. Relationships: is a type of GO:0065003; is part of transforming growth factor beta receptor signaling pathway [GO:0007179] Sources: GOC:jl, Wikipedia:TGF_beta_signaling_pathway